sterigmatocystin metabolic process [GO:0045460] (biological process) Also known as: sterigmatocystin metabolism References: PMID:10618248 Subtypes: sterigmatocystin biosynthetic process [GO:0045461], sterigmatocystin catabolic process [GO:0045574] Relationships: is a type of toxin metabolic process [GO:0009404] Definition: The chemical reactions and pathways involving sterigmatocystin, a carcinogenic mycotoxin produced in high yields by strains of the common molds.